host cell uropod [GO:0120026] (cellular component) Definition: A host cell membrane projection with related cytoskeletal components at the trailing edge of a cell in the process of migrating or being activated, found on the opposite side of the cell from the leading edge or immunological synapse, respectively. References: PMID:24965475 Also known as: host cell uropodium Relationships: is a type of host cell projection [GO:0044157]